response to reversine [GO:1901596] (biological process) Subtypes: cellular response to reversine [GO:0072764] Relationships: is a type of response to purine-containing compound [GO:0014074]; is a type of response to oxygen-containing compound [GO:1901700] Sources: GOC:TermGenie Definition: Any process that results in a change in state or activity of a cell or an organism (in terms of movement, secretion, enzyme production, gene expression, etc.) as a result of a reversine stimulus.